{
  "term_label": "phosphatidylinositol phosphate binding",
  "gene": "UniProtKB:Q92622",
  "gene_name": "Run domain Beclin-1-interacting and cysteine-rich domain-containing protein",
  "term_id": "GO:1901981",
  "gene_symbol": "RUBCN"
}